{
  "gene_name": "Transcription factor SOX-3",
  "gene_symbol": "SOX3",
  "term_label": "negative regulation of transcription by RNA polymerase II",
  "term_id": "GO:0000122",
  "gene": "UniProtKB:P41225"
}